{
  "gene": "UniProtKB:Q4G0X4",
  "gene_name": "BTB_POZ domain-containing protein KCTD21",
  "gene_symbol": "KCTD21",
  "term_id": "UNKNOWN:0003",
  "term_label": "Unknown cellular component"
}